{
  "gene": "UniProtKB:A0A087WVF3",
  "gene_symbol": "TBC1D3D",
  "term_label": "GTPase activator activity",
  "gene_name": "TBC1 domain family member 3D",
  "term_id": "GO:0005096"
}